response to hyperoxia [GO:0055093] (biological process) Sources: GOC:kmv Also known as: response to hyperoxic stress, response to increased oxygen tension Definition: Any process that results in a change in state or activity of a cell or an organism (in terms of movement, secretion, enzyme production, gene expression, etc.) as a result of a stimulus indicating increased oxygen tension. Subtypes: cellular response to hyperoxia [GO:0071455] Relationships: is a type of response to stress [GO:0006950]; is a type of GO:0036296